negative regulation of natural killer cell mediated cytotoxicity [GO:0045953] (biological process) Also known as: down regulation of natural killer cell mediated cytotoxicity, down-regulation of natural killer cell mediated cytotoxicity, downregulation of natural killer cell mediated cytotoxicity, negative regulation of NK cell mediated cell death, negative regulation of NK cell mediated cell killing, negative regulation of NK cell mediated cytotoxicity, negative regulation of natural killer cell mediated cell death, negative regulation of natural killer cell mediated cell killing, inhibition of natural killer cell mediated cytotoxicity, negative regulation of NK cell mediated cytolysis, negative regulation of natural killer cell mediated cytolysis Relationships: is a type of negative regulation of leukocyte mediated cytotoxicity [GO:0001911]; is a type of negative regulation of natural killer cell mediated immunity [GO:0002716]; is a type of regulation of natural killer cell mediated cytotoxicity [GO:0042269]; negatively regulates natural killer cell mediated cytotoxicity [GO:0042267] Definition: Any process that stops, prevents, or reduces the rate of natural killer mediated cytotoxicity. Subtypes: negative regulation of natural killer cell mediated cytotoxicity directed against tumor cell target [GO:0002859], protection from natural killer cell mediated cytotoxicity [GO:0042270], negative regulation of natural killer cell degranulation [GO:0043322] Sources: GOC:add, ISBN:0781735149